carboxylic acid transmembrane transport [GO:1905039] (biological process) Definition: The process in which carboxylic acid is transported across a membrane. Subtypes: shikimate transmembrane transport [GO:0015733], uronic acid transmembrane transport [GO:0015735], UDP-glucuronate transmembrane transport [GO:0015787], aspartate transmembrane transport [GO:0015810], creatine transmembrane transport [GO:0015881], L-ascorbic acid transmembrane transport [GO:0015882], pantothenate transmembrane transport [GO:0015887], GO:0033308, acetate transmembrane transport [GO:0035433], GO:0035524, tricarboxylic acid transmembrane transport [GO:0035674], lactate transmembrane transport [GO:0035873], aldarate transmembrane transport [GO:0042869], GO:0042873, D-alanine transmembrane transport [GO:0042941], GO:0042942, 2-keto-3-deoxygluconate transmembrane transport [GO:0046411], GO:0048473, ectoine transmembrane transport [GO:0051470], phosphoenolpyruvate-dependent mannosylglycerate phosphotransferase system [GO:0051476], succinate transmembrane transport [GO:0071422], malate transmembrane transport [GO:0071423], phosphoenolpyruvate transmembrane transport [GO:0089722], glutamate transmembrane import into vacuole [GO:0090454], ornithine transmembrane import into vacuole [GO:0090455], glycolate transmembrane transport [GO:0097339], serine import across plasma membrane [GO:0098718], folate transmembrane transport [GO:0098838], serine import into mitochondrion [GO:0140300], GO:0140484, pyruvate transmembrane transport [GO:1901475], GO:1901553, fatty acid transmembrane transport [GO:1902001], oxaloacetate(2-) transmembrane transport [GO:1902356], 2-isopropylmalate(2-) transmembrane transport [GO:1902357], L-alpha-amino acid transmembrane transport [GO:1902475], GO:1902604, quinolinic acid transmembrane transport [GO:1903222], GO:1903692, cysteine transmembrane transport [GO:1903712], GO:1903713, GO:1903714, glycine import across plasma membrane [GO:1903804], glycine import into mitochondrion [GO:1904983], biotin import across plasma membrane [GO:1905135], dethiobiotin import across plasma membrane [GO:1905136], gibberellic acid transmembrane transport [GO:1905200], GO:1990550, GO:1990551 References: PMID:10869563 Sources: GOC:TermGenie, GO_REF:0000069 Relationships: is a type of carboxylic acid transport [GO:0046942]; is a type of GO:0055085